sensory perception [GO:0007600] (biological process) Sources: GOC:ai, GOC:dph Relationships: is a type of nervous system process [GO:0050877] Definition: The series of events required for an organism to receive a sensory stimulus, convert it to a molecular signal, and recognize and characterize the signal. This is a neurological process. Regulation: RO_0002211 by regulation of sensory perception [GO:0051931] Subtypes: sensory perception of chemical stimulus [GO:0007606], proprioception [GO:0019230], sensory perception of pain [GO:0019233], sensory perception of temperature stimulus [GO:0050951], GO:0050952, sensory perception of light stimulus [GO:0050953], sensory perception of mechanical stimulus [GO:0050954], equilibrioception [GO:0050957], magnetoreception [GO:0050958], sensory perception of gravity [GO:0070998], sensory perception of humidity [GO:0098509], sensory perception of itch [GO:0160025]